{
  "gene_name": "Glucose-6-phosphate isomerase",
  "gene_symbol": "GPI",
  "term_label": "cytosol",
  "gene": "UniProtKB:P06744",
  "term_id": "GO:0005829"
}